Toll receptor ligand protein activation cascade [GO:0160032] (biological process) Relationships: is a type of protein activation cascade [GO:0072376]; has part signaling receptor ligand precursor processing [GO:0140448] Note: This term specifically mentions the Toll receptor and its ligand spatzle because this is the only known example of such an activation cascade for a ligand. Definition: A protein activation cascade that generates the active Toll receptor ligand and consists of the cascade of enzymatic reactions initiated by extracellular recognition factors, leading to the cleavage of the inactive form of spatzle family of ligands. References: PMID:23632253 Regulation: regulated by regulation of Toll receptor ligand protein activation cascade [GO:0160033]; positively regulated by positive regulation of Toll receptor ligand protein activation cascade [GO:0160034]; negatively regulated by GO:0160035